{
  "term_label": "Unknown cellular component",
  "term_id": "UNKNOWN:0003",
  "gene_name": "Ras GTPase-activating protein 4B",
  "gene": "UniProtKB:C9J798",
  "gene_symbol": "RASA4B"
}